regulation of preblastoderm mitotic cell cycle [GO:0007347] (biological process) Sources: GOC:dph, GOC:go_curators, GOC:tb Also known as: modulation of preblastoderm mitotic cell cycle progression, preblastoderm mitotic cell cycle modulation, preblastoderm mitotic cell cycle regulation, regulation of preblastoderm mitotic cell cycle progression, regulation of progression through preblastoderm mitotic cell cycle, preblastoderm mitotic cell cycle regulator Subtypes: negative regulation of preblastoderm mitotic cell cycle [GO:0046001], positive regulation of preblastoderm mitotic cell cycle [GO:0046002] Definition: A cell cycle process that modulates the rate or extent of the progression through the preblastoderm mitotic cell cycle. Relationships: is_a regulation of mitotic cell cycle, embryonic [GO:0009794]; regulates GO:0035185